{
  "gene_name": "Small integral membrane protein 2",
  "term_id": "UNKNOWN:0003",
  "term_label": "Unknown cellular component",
  "gene": "UniProtKB:Q9BVW6",
  "gene_symbol": "SMIM2"
}